{
  "gene_symbol": "ZZEF1",
  "term_label": "Unknown biological process",
  "gene": "UniProtKB:O43149",
  "gene_name": "Zinc finger ZZ-type and EF-hand domain-containing protein 1",
  "term_id": "UNKNOWN:0002"
}